kinetoplast DNA replication [GO:0140909] (biological process) Definition: The process of doubling of the number of maxicircles and minicircles and distribution of the progeny into two daughter networks, which are identical to the parent kinetoplast DNA network. Also known as: kDNA replication, kinetoplast DNA synthesis, replication of kinetoplast DNA Relationships: is a type of mitochondrial DNA replication [GO:0006264]; occurs in kinetoplast [GO:0020023] References: PMID:12455998, PMID:15967722, PMID:17462016, PMID:8045928, PMID:8561456 Sources: GOC:ach